{
  "term_id": "GO:0043005",
  "gene": "UniProtKB:P30874",
  "gene_symbol": "SSTR2",
  "term_label": "neuron projection",
  "gene_name": "Somatostatin receptor type 2"
}